{
  "gene_name": "Small ribosomal subunit protein uS8",
  "term_label": "structural constituent of ribosome",
  "term_id": "GO:0003735",
  "gene_symbol": "RPS15A",
  "gene": "UniProtKB:P62244"
}